{
  "gene_name": "Rab15 effector protein",
  "gene": "UniProtKB:Q6BDI9",
  "term_label": "endosome membrane",
  "gene_symbol": "REP15",
  "term_id": "GO:0010008"
}